L-alanine transport [GO:0015808] (biological process) Sources: GOC:ai, GOC:jsg, GOC:mah Relationships: is a type of L-amino acid transport [GO:0015807]; is a type of GO:0032328 Definition: The directed movement of L-alanine, the L-enantiomer of 2-aminopropanoic acid, into, out of or within a cell, or between cells, by means of some agent such as a transporter or pore. Subtypes: L-alanine transmembrane transport [GO:1904557]